{
  "term_id": "GO:0000785",
  "gene_symbol": "TSPYL6",
  "gene_name": "Testis-specific Y-encoded-like protein 6",
  "gene": "UniProtKB:Q8N831",
  "term_label": "chromatin"
}